{
  "gene_symbol": "BCL6",
  "term_id": "GO:0005654",
  "gene": "UniProtKB:P41182",
  "gene_name": "B-cell lymphoma 6 protein",
  "term_label": "nucleoplasm"
}